{
  "gene": "UniProtKB:Q9H4I8",
  "term_id": "GO:0016787",
  "term_label": "hydrolase activity",
  "gene_name": "Serine hydrolase-like protein 2",
  "gene_symbol": "SERHL2"
}